positive regulation of Toll signaling pathway [GO:0045752] (biological process) Definition: Any process that activates or increases the frequency, rate or extent of the Tl signaling pathway. Sources: GOC:go_curators Relationships: is a type of regulation of Toll signaling pathway [GO:0008592]; is a type of positive regulation of signal transduction [GO:0009967]; positively regulates GO:0008063 Also known as: positive regulation of Tl signaling pathway, positive regulation of Tl signalling pathway, up regulation of Toll signaling pathway, up-regulation of Toll signaling pathway, upregulation of Toll signaling pathway, activation of Toll signaling pathway, stimulation of Toll signaling pathway